{
  "term_id": "GO:0005262",
  "gene": "UniProtKB:Q8NE86",
  "term_label": "calcium channel activity",
  "gene_symbol": "MCU",
  "gene_name": "Calcium uniporter protein, mitochondrial"
}